{
  "term_id": "GO:0045211",
  "gene_symbol": "SHANK1",
  "term_label": "postsynaptic membrane",
  "gene_name": "SH3 and multiple ankyrin repeat domains protein 1",
  "gene": "UniProtKB:Q9Y566"
}